{
  "term_label": "Unknown biological process",
  "gene_symbol": "SPRING1",
  "gene_name": "SREBP regulating gene protein",
  "term_id": "UNKNOWN:0002",
  "gene": "UniProtKB:Q9H741"
}